{
  "term_id": "UNKNOWN:0001",
  "gene": "UniProtKB:Q7Z7A4",
  "gene_name": "PX domain-containing protein kinase-like protein",
  "term_label": "Unknown molecular function",
  "gene_symbol": "PXK"
}